{
  "gene_name": "Dual specificity protein phosphatase 13 isoform B",
  "term_label": "protein tyrosine/serine/threonine phosphatase activity",
  "term_id": "GO:0008138",
  "gene_symbol": "DUSP13B",
  "gene": "UniProtKB:Q9UII6"
}